{
  "term_id": "UNKNOWN:0001",
  "gene_name": "Gliomedin",
  "term_label": "Unknown molecular function",
  "gene_symbol": "GLDN",
  "gene": "UniProtKB:Q6ZMI3"
}